{
  "gene_name": "Vascular endothelial growth factor A, long form",
  "term_label": "vascular endothelial growth factor receptor binding",
  "gene_symbol": "VEGFA",
  "gene": "UniProtKB:P15692",
  "term_id": "GO:0005172"
}